{
  "gene": "UniProtKB:Q99958",
  "term_label": "anatomical structure morphogenesis",
  "gene_symbol": "FOXC2",
  "term_id": "GO:0009653",
  "gene_name": "Forkhead box protein C2"
}